skeletal muscle satellite cell proliferation [GO:0014841] (BP) Regulation: regulated by regulation of skeletal muscle satellite cell proliferation [GO:0014842]; negatively regulated by negative regulation of skeletal muscle satellite cell proliferation [GO:1902723]; positively regulated by positive regulation of skeletal muscle satellite cell proliferation [GO:1902724] References: PMID:16607119 Sources: GOC:ef, GOC:mtg_muscle Relationships: is a type of GO:0014856 Definition: The multiplication or reproduction of satellite cells, resulting in the expansion of the cell population. Satellite cells are quiescent cells that are located between the basal lamina and the plasmalemma of the muscle fiber, which are the main contributors to postnatal muscle growth. In adult muscle, satellite cells become activated to divide and differentiate in response to muscle damage.